{
  "term_id": "GO:0008104",
  "gene_symbol": "SEPTIN5",
  "gene_name": "Septin-5",
  "term_label": "intracellular protein localization",
  "gene": "UniProtKB:Q99719"
}